{
  "term_id": "GO:0030141",
  "gene_name": "Serine protease 58",
  "term_label": "secretory granule",
  "gene_symbol": "PRSS58",
  "gene": "UniProtKB:Q8IYP2"
}